orexin secretion [GO:0061584] (biological process) Relationships: is a type of GO:0002790 Also known as: hypocretin secretion Subtypes: orexin secretion, neurotransmission [GO:0061585] Definition: The controlled release of orexin from a cell or a tissue. Sources: GOC:dph